{
  "term_label": "GTPase activator activity",
  "term_id": "GO:0005096",
  "gene": "UniProtKB:Q92619",
  "gene_name": "Rho GTPase-activating protein 45",
  "gene_symbol": "ARHGAP45"
}